{
  "term_id": "GO:1901907",
  "gene": "UniProtKB:O95989",
  "term_label": "diadenosine pentaphosphate catabolic process",
  "gene_symbol": "NUDT3",
  "gene_name": "Diphosphoinositol polyphosphate phosphohydrolase 1"
}